DAPK1-calmodulin complex [GO:1990722] (cellular component) Definition: A serine/threonine protein kinase complex involved in cell survival, apoptosis and autophagic cell death pathways. DAPK1 is activated by the dephosphorylation of a n-terminal serine and calcium-calmodulin binding. Relationships: is a type of GO:1902554 Also known as: death-associated protein kinase 1 - calmodulin complex References: PMID:20103772 Sources: GOC:bhm